protein side chain deglutamylation [GO:0035610] (biological process) References: PMID:21074048 Sources: GOC:sp Definition: The removal of a glutamate residue from the side chain of a protein. Glutamate side chains are added to glutamic acid residues within the primary protein sequence during polyglutamylation. Also known as: removal of posttranslational polyglutamylation, shortening of glutamate side chain Relationships: is a type of GO:0035608